{
  "gene_name": "Transmembrane protein 276",
  "term_id": "UNKNOWN:0002",
  "gene_symbol": "TMEM276",
  "term_label": "Unknown biological process",
  "gene": "UniProtKB:P0DTL5"
}